{
  "gene": "UniProtKB:O75352",
  "term_label": "Unknown molecular function",
  "gene_symbol": "MPDU1",
  "term_id": "UNKNOWN:0001",
  "gene_name": "Mannose-P-dolichol utilization defect 1 protein"
}